determination of adult lifespan [GO:0008340] (biological process) References: PMID:25561524, PMID:273723695, PMID:3424805 Relationships: is a type of multicellular organismal process [GO:0032501] Definition: The pathways that regulate the duration of the adult phase of the life-cycle of an animal.